{
  "term_label": "3',5'-cyclic-AMP phosphodiesterase activity",
  "gene_name": "High affinity cAMP-specific 3',5'-cyclic phosphodiesterase 7A",
  "term_id": "GO:0004115",
  "gene_symbol": "PDE7A",
  "gene": "UniProtKB:Q13946"
}